{
  "gene_name": "Thioredoxin, mitochondrial",
  "gene_symbol": "TXN2",
  "term_id": "GO:0045454",
  "term_label": "cell redox homeostasis",
  "gene": "UniProtKB:Q99757"
}